{
  "gene_symbol": "ZNF331",
  "gene_name": "Zinc finger protein 331",
  "term_id": "GO:0000978",
  "term_label": "RNA polymerase II cis-regulatory region sequence-specific DNA binding",
  "gene": "UniProtKB:Q9NQX6"
}